{
  "term_label": "neuron projection development",
  "gene_name": "G protein-regulated inducer of neurite outgrowth 1",
  "term_id": "GO:0031175",
  "gene_symbol": "GPRIN1",
  "gene": "UniProtKB:Q7Z2K8"
}